aldose 1-epimerase activity [GO:0004034] (MF) Definition: Catalysis of the reaction: alpha-D-glucose = beta-D-glucose. Also acts on L-arabinose, D-xylose, D-galactose, maltose and lactose. Also known as: aldose mutarotase activity, mutarotase activity Sources: EC:5.1.3.3 Relationships: is a type of racemase and epimerase activity, acting on carbohydrates and derivatives [GO:0016857]